{
  "term_label": "extracellular space",
  "gene_symbol": "F9",
  "gene": "UniProtKB:P00740",
  "gene_name": "Coagulation factor IX",
  "term_id": "GO:0005615"
}